{
  "gene": "UniProtKB:O15355",
  "gene_name": "Protein phosphatase 1G",
  "gene_symbol": "PPM1G",
  "term_id": "GO:0004722",
  "term_label": "protein serine/threonine phosphatase activity"
}